{
  "term_label": "Unknown biological process",
  "gene_symbol": "DNAJC21",
  "gene": "UniProtKB:Q5F1R6",
  "gene_name": "DnaJ homolog subfamily C member 21",
  "term_id": "UNKNOWN:0002"
}